quercetin catabolic process [GO:1901733] (biological process) Relationships: is_a flavonoid catabolic process [GO:0046275]; is a type of GO:0051552 Sources: GOC:TermGenie, GOC:yaf, UniPathway:UPA00724 Also known as: quercetin breakdown, quercetin catabolism, quercetin degradation Definition: The chemical reactions and pathways resulting in the breakdown of quercetin.